{
  "gene": "UniProtKB:Q2TAY7",
  "gene_symbol": "SMU1",
  "gene_name": "WD40 repeat-containing protein SMU1",
  "term_id": "UNKNOWN:0001",
  "term_label": "Unknown molecular function"
}